histone H3K14 deacetylase activity, hydrolytic mechanism [GO:0031078] (molecular function) Relationships: is a type of histone H3K deacetylase activity [GO:0141050]; is a type of histone deacetylase activity, hydrolytic mechanism [GO:0141221] Also known as: histone H3K14 deacetylase activity, histone H3-K14 deacetylase activity, histone deacetylase activity (H3-K14 specific) Definition: Catalysis of the reaction: histone H3 N6-acetyl-L-lysine (position 14) + H2O = histone H3 L-lysine (position 14) + acetate. This reaction represents the removal of an acetyl group from lysine at position 14 of the histone H3 protein. Note: Comment: Note that the residue position corresponds to the canonical human H3 histone (UniProtKB:P84243); this residue is conserved across all eukaryotes. Residue 1 is the first residue following removal of the initiating Methionine (Met). Note that each histone is encoded by multiple genes, and sequences may vary across different genes within an organism. References: PMID:28450737